{
  "term_id": "GO:0051489",
  "gene_name": "Protein Abitram",
  "gene_symbol": "ABITRAM",
  "term_label": "regulation of filopodium assembly",
  "gene": "UniProtKB:Q9NX38"
}